{
  "term_label": "negative regulation of transcription by RNA polymerase II",
  "gene_name": "Unconventional prefoldin RPB5 interactor 1",
  "term_id": "GO:0000122",
  "gene_symbol": "URI1",
  "gene": "UniProtKB:O94763"
}